double-stranded DNA 3'-5' DNA exonuclease activity [GO:0008311] (molecular function) References: PMID:22562358 Sources: GOC:mah Also known as: double-stranded DNA 3'-5' exodeoxyribonuclease activity, exonuclease III activity, exoribonuclease III activity, double-stranded DNA specific 3'-5' exodeoxyribonuclease activity Definition: Catalysis of the sequential cleavage of mononucleotides from a free 3' terminus of a double-stranded DNA molecule. Relationships: is a type of GO:0008296; is a type of double-stranded DNA exodeoxyribonuclease activity [GO:0008309]